tubovesicular membrane network [GO:0085026] (cellular component) Relationships: is a type of host cell cytoplasm part [GO:0033655]; is a type of extracellular membraneless organelle [GO:0043264] Definition: A complex, symbiont-induced host-derived organelle that is comprised of multiple protein and lipid domains. Sources: GOC:pamgo_curators Also known as: TVM network, TVN